{
  "gene_name": "Beta-defensin 129",
  "term_label": "Unknown molecular function",
  "gene_symbol": "DEFB129",
  "gene": "UniProtKB:Q9H1M3",
  "term_id": "UNKNOWN:0001"
}